{
  "term_id": "UNKNOWN:0003",
  "gene": "UniProtKB:Q9H0W8",
  "gene_name": "Nonsense-mediated mRNA decay factor SMG9",
  "gene_symbol": "SMG9",
  "term_label": "Unknown cellular component"
}